cellular response to reactive nitrogen species [GO:1902170] (biological process) Relationships: is a type of cellular response to nitrogen compound [GO:1901699] References: PMID:22504638 Sources: GOC:TermGenie, GOC:sl Definition: Any process that results in a change in state or activity of a cell (in terms of movement, secretion, enzyme production, gene expression, etc.) as a result of a reactive nitrogen species stimulus. Subtypes: cellular response to nitrate [GO:0071249], cellular response to nitrite [GO:0071250], GO:0071732